{
  "gene_symbol": "ZC3H12C",
  "gene_name": "Probable ribonuclease ZC3H12C",
  "term_label": "cytoplasmic ribonucleoprotein granule",
  "gene": "UniProtKB:Q9C0D7",
  "term_id": "GO:0036464"
}